{
  "gene_symbol": "CCDC88A",
  "term_id": "GO:0005737",
  "gene_name": "Girdin",
  "gene": "UniProtKB:Q3V6T2",
  "term_label": "cytoplasm"
}